NADH dehydrogenase (ubiquinone) activity [GO:0008137] (molecular function) Definition: Catalysis of the reaction: NADH + ubiquinone + 5 H+(in) = NAD+ + ubiquinol + 4 H+(out). Also known as: ubiquinone reductase activity, mitochondrial electron transport complex 1 activity, mitochondrial electron transport complex I activity, DPNH-coenzyme Q reductase activity, DPNH-ubiquinone reductase activity, NADH coenzyme Q1 reductase activity, NADH-CoQ oxidoreductase activity, NADH-CoQ reductase activity, NADH-Q6 oxidoreductase activity, NADH-coenzyme Q oxidoreductase activity, NADH-coenzyme Q reductase activity, NADH-ubiquinone oxidoreductase activity, NADH-ubiquinone reductase activity, NADH-ubiquinone-1 reductase activity, NADH:ubiquinone oxidoreductase activity, NADH:ubiquinone oxidoreductase complex activity, coenzyme Q reductase activity, complex 1 dehydrogenase activity, complex I (NADH:Q1 oxidoreductase) activity, complex I (electron transport chain) activity, complex I (mitochondrial electron transport) activity, dihydronicotinamide adenine dinucleotide-coenzyme Q reductase activity, electron transfer complex I activity, reduced nicotinamide adenine dinucleotide-coenzyme Q reductase activity, type 1 dehydrogenase activity Relationships: is a type of electron transfer activity [GO:0009055]; is a type of GO:0015078; is a type of oxidoreduction-driven active transmembrane transporter activity [GO:0015453]; is a type of GO:0022853; BFO_0000051 GO:0003954; has part GO:0016655 Sources: RHEA:29091